{
  "term_label": "nuclear-transcribed mRNA catabolic process, deadenylation-dependent decay",
  "gene_name": "Roquin-1",
  "term_id": "GO:0000288",
  "gene": "UniProtKB:Q5TC82",
  "gene_symbol": "RC3H1"
}